{
  "gene_name": "Fibroblast growth factor 2",
  "gene_symbol": "FGF2",
  "term_id": "GO:0030334",
  "term_label": "regulation of cell migration",
  "gene": "UniProtKB:P09038"
}